ganglioside GM3 binding [GO:1905575] (molecular function) References: PMID:1454804 Sources: GOC:TermGenie, GO_REF:0000067 Relationships: is a type of monocarboxylic acid binding [GO:0033293]; is a type of GO:0035594 Definition: Binding to ganglioside GM3.